transcription factor binding [GO:0008134] (molecular function) Relationships: is_a GO:0005515 Subtypes: transcription coregulator binding [GO:0001221], GO:0140296, DNA-binding transcription factor binding [GO:0140297] Note: Note that this term should not be used for direct annotation. Please consider one of the more specific descendants, GO:0140297 ; DNA-binding transcription factor binding, GO:0140296 ; general transcription initiation factor binding or GO:0001221 ; transcription coregulator binding. Also known as: TF binding, transcription regulator binding Sources: ISBN:0198506732 Definition: Binding to a transcription factor, a protein required to initiate or regulate transcription.